{
  "gene_symbol": "KRTAP10-5",
  "term_id": "UNKNOWN:0001",
  "term_label": "Unknown molecular function",
  "gene_name": "Keratin-associated protein 10-5",
  "gene": "UniProtKB:P60370"
}